{
  "gene_name": "Charged multivesicular body protein 4b",
  "gene_symbol": "CHMP4B",
  "term_id": "GO:0031468",
  "term_label": "nuclear membrane reassembly",
  "gene": "UniProtKB:Q9H444"
}